positive regulation of formation of translation preinitiation complex [GO:1901195] (BP) Also known as: activation of formation of translation pre-initiation complex, activation of translation preinitiation complex assembly, positive regulation of formation of translation pre-initiation complex, positive regulation of translation preinitiation complex assembly, up regulation of formation of translation pre-initiation complex, up regulation of formation of translation preinitiation complex, up regulation of translation preinitiation complex assembly, up-regulation of formation of translation pre-initiation complex, up-regulation of formation of translation preinitiation complex, up-regulation of translation preinitiation complex assembly, upregulation of formation of translation pre-initiation complex, upregulation of formation of translation preinitiation complex, upregulation of translation preinitiation complex assembly, activation of formation of translation preinitiation complex Relationships: is a type of positive regulation of protein-containing complex assembly [GO:0031334]; is a type of regulation of formation of translation preinitiation complex [GO:1901193]; positively regulates formation of translation preinitiation complex [GO:0001731] Definition: Any process that activates or increases the frequency, rate or extent of formation of translation preinitiation complex. Sources: GOC:TermGenie